{
  "term_id": "GO:0070652",
  "gene_symbol": "HAUS2",
  "gene": "UniProtKB:Q9NVX0",
  "term_label": "HAUS complex",
  "gene_name": "HAUS augmin-like complex subunit 2"
}